acetylajmaline esterase activity [GO:0033879] (molecular function) Relationships: is a type of GO:0052689 Sources: EC:3.1.1.80 Also known as: 17-O-acetylajmaline O-acetylhydrolase activity, 2beta(R)-17-O-acetylajmalan:acetylesterase activity, AAE, acetylajmalan esterase activity Definition: Catalysis of the reactions: 17-O-acetylajmaline + H2O = ajmaline + acetate, and 17-O-acetylnorajmaline + H2O = norajmaline + acetate.